{
  "term_id": "UNKNOWN:0002",
  "gene_name": "Sucrase-isomaltase, intestinal",
  "gene": "UniProtKB:P14410",
  "gene_symbol": "SI",
  "term_label": "Unknown biological process"
}